{
  "term_id": "GO:1990756",
  "term_label": "ubiquitin-like ligase-substrate adaptor activity",
  "gene": "UniProtKB:Q5VXH5",
  "gene_name": "PRAME family member 7",
  "gene_symbol": "PRAMEF7"
}